COPII vesicle coat [GO:0030127] (cellular component) Relationships: is_a vesicle coat [GO:0030120]; is part of GO:0012507 References: PMID:11252894 Sources: GOC:ascb_2009, GOC:dph, GOC:mah, GOC:tb Definition: One of two multimeric complexes that forms a membrane vesicle coat. COPII is best characterized in S. cerevisiae, where the subunits are called Sar1p, Sec13p, Sec31p, Sec23p, and Sec24p. Vesicles with COPII coats are found associated with endoplasmic reticulum (ER) membranes at steady state.